{
  "gene_symbol": "FGFR3",
  "term_label": "positive regulation of MAPK cascade",
  "gene_name": "Fibroblast growth factor receptor 3",
  "gene": "UniProtKB:P22607",
  "term_id": "GO:0043410"
}